{
  "gene_name": "ATP-binding cassette sub-family A member 13",
  "term_id": "GO:0006869",
  "term_label": "lipid transport",
  "gene_symbol": "ABCA13",
  "gene": "UniProtKB:Q86UQ4"
}